{
  "gene": "UniProtKB:Q12929",
  "gene_name": "Epidermal growth factor receptor kinase substrate 8",
  "term_id": "GO:0032587",
  "gene_symbol": "EPS8",
  "term_label": "ruffle membrane"
}